{
  "term_id": "GO:0005615",
  "gene": "UniProtKB:P08185",
  "gene_symbol": "SERPINA6",
  "gene_name": "Corticosteroid-binding globulin",
  "term_label": "extracellular space"
}